{
  "gene": "UniProtKB:Q8NBL1",
  "gene_symbol": "POGLUT1",
  "term_label": "protein O-linked glycosylation",
  "term_id": "GO:0006493",
  "gene_name": "Protein O-glucosyltransferase 1"
}